negative regulation of methane biosynthetic process from formic acid [GO:1900340] (biological process) Definition: Any process that stops, prevents or reduces the frequency, rate or extent of methane biosynthetic process from formic acid. Relationships: is a type of negative regulation of small molecule metabolic process [GO:0062014]; is a type of regulation of methane biosynthetic process from formic acid [GO:1900339]; is a type of GO:1901578; is a type of negative regulation of cellular respiration [GO:1901856]; negatively regulates methane biosynthetic process from formic acid [GO:2001127] Sources: GOC:TermGenie, GOC:mengo_curators Also known as: down regulation of methane biosynthetic process from formic acid, down-regulation of methane biosynthetic process from formic acid, downregulation of methane biosynthetic process from formic acid, inhibition of methane biosynthetic process from formic acid